{
  "gene": "UniProtKB:P35503",
  "term_label": "enzyme binding",
  "term_id": "GO:0019899",
  "gene_name": "UDP-glucuronosyltransferase 1A3",
  "gene_symbol": "UGT1A3"
}